{
  "term_label": "siRNA processing",
  "gene_symbol": "DICER1",
  "gene_name": "Endoribonuclease Dicer",
  "term_id": "GO:0030422",
  "gene": "UniProtKB:Q9UPY3"
}